selenide, water dikinase activity [GO:0004756] (molecular function) Also known as: selenophosphate synthase activity, ATP:selenide, water phosphotransferase activity, selenide,water dikinase activity, selenium donor protein activity, selenophosphate synthetase activity Sources: EC:2.7.9.3, RHEA:18737 Relationships: is a type of kinase activity [GO:0016301]; is_a phosphotransferase activity, paired acceptors [GO:0016781] Definition: Catalysis of the reaction: ATP + H2O + hydrogen selenide = AMP + 3 H+ + phosphate + selenophosphorate.